{
  "term_label": "plasma membrane",
  "gene_name": "ATP-sensitive inward rectifier potassium channel 10",
  "gene_symbol": "KCNJ10",
  "term_id": "GO:0005886",
  "gene": "UniProtKB:P78508"
}